{
  "term_label": "phospholipid binding",
  "gene": "UniProtKB:P49418",
  "gene_name": "Amphiphysin",
  "gene_symbol": "AMPH",
  "term_id": "GO:0005543"
}